single-stranded DNA-binding protein complex [GO:0044777] (cellular component) Definition: A homotetrameric protein complex that is essential for DNA replication. It supercoils the single-stranded DNA preventing DNA duplexing before the polymerase holoenzyme passes and synthesizes the complementary strand. It is also involved in DNA recombination and repair. Sources: GOC:jl, UniProt:P0AGE0 Also known as: SSB complex Relationships: is a type of protein-containing complex [GO:0032991]; is part of nucleoid [GO:0009295]